{
  "term_label": "RNA uridylyltransferase activity",
  "gene": "UniProtKB:Q5VYS8",
  "gene_name": "Terminal uridylyltransferase 7",
  "gene_symbol": "TUT7",
  "term_id": "GO:0050265"
}